{
  "gene_symbol": "ZNF865",
  "gene": "UniProtKB:P0CJ78",
  "gene_name": "Zinc finger protein 865",
  "term_label": "RNA polymerase II cis-regulatory region sequence-specific DNA binding",
  "term_id": "GO:0000978"
}